regulation of viral entry into host cell [GO:0046596] (biological process) Relationships: is a type of GO:0052372; is a type of regulation of viral life cycle [GO:1903900]; regulates symbiont entry into host cell [GO:0046718] Definition: Any process that modulates the frequency, rate or extent of the viral entry into the host cell. Sources: GOC:jl Subtypes: positive regulation of viral entry into host cell [GO:0046598], regulation of fusion of virus membrane with host plasma membrane [GO:1903913] Also known as: regulation of viral penetration into host cell, viral escort protein